{
  "term_id": "GO:0046825",
  "gene_name": "Serine_threonine-protein kinase Kist",
  "gene_symbol": "UHMK1",
  "gene": "UniProtKB:Q8TAS1",
  "term_label": "regulation of protein export from nucleus"
}